{
  "gene": "UniProtKB:O75208",
  "gene_symbol": "COQ9",
  "gene_name": "Ubiquinone biosynthesis protein COQ9, mitochondrial",
  "term_id": "GO:0005743",
  "term_label": "mitochondrial inner membrane"
}